regulation of macrophage colony-stimulating factor signaling pathway [GO:1902226] (biological process) Definition: Any process that modulates the frequency, rate or extent of macrophage colony-stimulating factor signaling pathway. References: PMID:16705167 Sources: GOC:TermGenie Also known as: regulation of M-CSF signaling pathway, regulation of macrophage colony-stimulating factor signalling pathway Relationships: is a type of regulation of cytokine-mediated signaling pathway [GO:0001959]; is a type of regulation of cellular response to macrophage colony-stimulating factor stimulus [GO:1903972]; regulates macrophage colony-stimulating factor signaling pathway [GO:0038145] Subtypes: negative regulation of macrophage colony-stimulating factor signaling pathway [GO:1902227], positive regulation of macrophage colony-stimulating factor signaling pathway [GO:1902228]